{
  "term_label": "sulfur compound metabolic process",
  "gene_name": "Carbohydrate sulfotransferase 6",
  "gene": "UniProtKB:Q9GZX3",
  "term_id": "GO:0006790",
  "gene_symbol": "CHST6"
}